{
  "term_label": "regulation of proteolysis",
  "term_id": "GO:0030162",
  "gene_symbol": "RHOBTB3",
  "gene": "UniProtKB:O94955",
  "gene_name": "Rho-related BTB domain-containing protein 3"
}